{
  "gene_symbol": "RHOF",
  "gene_name": "Rho-related GTP-binding protein RhoF",
  "gene": "UniProtKB:Q9HBH0",
  "term_id": "GO:0005829",
  "term_label": "cytosol"
}